{
  "term_label": "positive regulation of cell population proliferation",
  "gene_symbol": "FGF10",
  "term_id": "GO:0008284",
  "gene": "UniProtKB:O15520",
  "gene_name": "Fibroblast growth factor 10"
}